{
  "gene": "UniProtKB:A6NDN3",
  "term_id": "GO:0032580",
  "gene_name": "Golgin subfamily A member 6B",
  "term_label": "Golgi cisterna membrane",
  "gene_symbol": "GOLGA6B"
}